{
  "term_id": "UNKNOWN:0001",
  "gene_name": "WD repeat-containing protein 62",
  "gene_symbol": "WDR62",
  "gene": "UniProtKB:O43379",
  "term_label": "Unknown molecular function"
}